{
  "gene": "UniProtKB:Q8N4B1",
  "term_label": "recycling endosome",
  "gene_name": "Sesquipedalian-1",
  "gene_symbol": "PHETA1",
  "term_id": "GO:0055037"
}